bacteriochlorophyll c binding [GO:0016169] (molecular function) Relationships: is a type of bacteriochlorophyll binding [GO:0042314] Definition: Binding to bacteriochlorophyll c, a chlorophyll of photosynthetic bacteria, for example green sulfur bacteria. Sources: ISBN:0192800981